{
  "gene_name": "Protein C-ets-2",
  "term_label": "DNA-binding transcription factor activity, RNA polymerase II-specific",
  "gene_symbol": "ETS2",
  "term_id": "GO:0000981",
  "gene": "UniProtKB:P15036"
}